{
  "term_id": "GO:0005737",
  "gene_symbol": "PIH1D1",
  "gene_name": "PIH1 domain-containing protein 1",
  "term_label": "cytoplasm",
  "gene": "UniProtKB:Q9NWS0"
}